{
  "gene": "UniProtKB:Q9GZM8",
  "gene_name": "Nuclear distribution protein nudE-like 1",
  "term_label": "vesicle transport along microtubule",
  "term_id": "GO:0047496",
  "gene_symbol": "NDEL1"
}